uronic acid transmembrane transporter activity [GO:0015133] (molecular function) Definition: Enables the transfer of uronic acid from one side of a membrane to the other. Uronic acids are any monocarboxylic acid formally derived by oxidizing to a carboxyl group the terminal hydroxymethylene group of either an aldose with four or more carbon atoms in the molecule, or of any glycoside derived from such an aldose. Subtypes: hexuronate transmembrane transporter activity [GO:0015134] Sources: GOC:ai Relationships: is a type of monocarboxylic acid transmembrane transporter activity [GO:0008028]; is a type of monosaccharide transmembrane transporter activity [GO:0015145]; is part of uronic acid transmembrane transport [GO:0015735]